{
  "term_label": "Unknown molecular function",
  "gene_name": "Transmembrane protein 59",
  "gene_symbol": "TMEM59",
  "gene": "UniProtKB:Q9BXS4",
  "term_id": "UNKNOWN:0001"
}